anterior commissure morphogenesis [GO:0021960] (biological process) Sources: GOC:cls, GOC:dgh, GOC:dph, GOC:jid, GO_REF:0000021 Relationships: is a type of central nervous system projection neuron axonogenesis [GO:0021952]; is part of telencephalon development [GO:0021537] Definition: Generation of a long process of a CNS neuron, that carries efferent (outgoing) action potentials from the cell body in one half of the cerebral cortex towards target cells in the contralateral half. This axonal process is a member of those that make up the anterior commissure, a small midline fiber tract that lies at the anterior end of the corpus callosum.